{
  "gene_symbol": "AHRR",
  "gene": "UniProtKB:A9YTQ3",
  "term_label": "nucleus",
  "gene_name": "Aryl hydrocarbon receptor repressor",
  "term_id": "GO:0005634"
}